{
  "term_id": "UNKNOWN:0001",
  "term_label": "Unknown molecular function",
  "gene_symbol": "SLC22A20P",
  "gene_name": "Solute carrier family 22 member 20",
  "gene": "UniProtKB:A6NK97"
}